{
  "gene_name": "Cholesteryl ester transfer protein",
  "gene": "UniProtKB:P11597",
  "term_label": "triglyceride binding",
  "term_id": "GO:0017129",
  "gene_symbol": "CETP"
}